{
  "term_id": "GO:0002009",
  "gene_symbol": "KRT36",
  "gene_name": "Keratin, type I cuticular Ha6",
  "gene": "UniProtKB:O76013",
  "term_label": "morphogenesis of an epithelium"
}